{
  "term_id": "GO:0000981",
  "gene": "UniProtKB:P09067",
  "term_label": "DNA-binding transcription factor activity, RNA polymerase II-specific",
  "gene_name": "Homeobox protein Hox-B5",
  "gene_symbol": "HOXB5"
}